{
  "gene_symbol": "RPS27A",
  "term_id": "GO:0019941",
  "gene_name": "Ubiquitin-ribosomal protein eS31 fusion protein",
  "term_label": "modification-dependent protein catabolic process",
  "gene": "UniProtKB:P62979"
}